{
  "gene_name": "Ras-related protein Rab-33A",
  "term_label": "endosome",
  "gene": "UniProtKB:Q14088",
  "term_id": "GO:0005768",
  "gene_symbol": "RAB33A"
}